{
  "gene": "UniProtKB:Q15742",
  "gene_name": "NGFI-A-binding protein 2",
  "term_id": "GO:0006355",
  "gene_symbol": "NAB2",
  "term_label": "regulation of DNA-templated transcription"
}